{
  "gene": "UniProtKB:Q96D09",
  "gene_name": "G-protein coupled receptor-associated sorting protein 2",
  "term_id": "GO:0005634",
  "gene_symbol": "GPRASP2",
  "term_label": "nucleus"
}